UBC13-MMS2 complex [GO:0031372] (cellular component) Definition: A heterodimeric ubiquitin conjugating enzyme complex that catalyzes assembly of K63-linked polyubiquitin chains. In Saccharomyces cerevisiae, the complex comprises Ubc13p and Mms2p; in human it comprises UBE2N and UBE2V1/UBE2V2; and in plants UBC35/UBC36 and UEV1A/UEV1B/UEV1C/UEV1D-4. References: PMID:15772086, PMID:16129784 Sources: GOC:sjm Relationships: is a type of ubiquitin conjugating enzyme complex [GO:0031371] Also known as: BEN-UEV1A complex, UBE2N/UBE2NL complex, UBE2V1/UBE2V2 complex, Uev1A-ben complex, ubc-13-uev-1 complex